{
  "gene_name": "Pre-B-cell leukemia transcription factor 3",
  "term_label": "positive regulation of transcription by RNA polymerase II",
  "gene_symbol": "PBX3",
  "term_id": "GO:0045944",
  "gene": "UniProtKB:P40426"
}